{
  "gene_name": "Tight junction protein ZO-1",
  "gene": "UniProtKB:Q07157",
  "term_id": "GO:0150105",
  "term_label": "protein localization to cell-cell junction",
  "gene_symbol": "TJP1"
}